potassium ion binding [GO:0030955] (molecular function) Relationships: is a type of alkali metal ion binding [GO:0031420] Definition: Binding to a potassium ion (K+). Sources: GOC:mah Also known as: K ion binding